{
  "gene_name": "Trafficking protein particle complex subunit 2B",
  "gene": "UniProtKB:P0DI82",
  "term_label": "endoplasmic reticulum to Golgi vesicle-mediated transport",
  "term_id": "GO:0006888",
  "gene_symbol": "TRAPPC2B"
}